{
  "gene_name": "Radial spoke head protein 4 homolog A",
  "term_label": "axoneme assembly",
  "term_id": "GO:0035082",
  "gene": "UniProtKB:Q5TD94",
  "gene_symbol": "RSPH4A"
}